response to kainic acid [GO:1904373] (biological process) Relationships: is a type of response to amino acid [GO:0043200]; is a type of GO:1901698; is a type of response to oxygen-containing compound [GO:1901700] References: PMID:17443789 Sources: GOC:TermGenie, GO_REF:0000071 Subtypes: cellular response to kainic acid [GO:1904374] Definition: Any process that results in a change in state or activity of a cell or an organism (in terms of movement, secretion, enzyme production, gene expression, etc.) as a result of a kainic acid stimulus.